sakuranetin 6-hydroxylase activity [GO:0102536] (molecular function) Definition: Catalysis of the reaction: (2S)-sakuranetin + O2 + reduced [NADPH--hemoprotein reductase] = (2S)-7-methylcarthamidin + H(+) + H2O + oxidized [NADPH--hemoprotein reductase]. Relationships: is a type of oxidoreductase activity, acting on paired donors, with incorporation or reduction of molecular oxygen, NAD(P)H as one donor, and incorporation of one atom of oxygen [GO:0016709] References: PMID:23184958 Sources: RHEA:73431